{
  "term_id": "UNKNOWN:0001",
  "gene": "UniProtKB:Q9UHX1",
  "term_label": "Unknown molecular function",
  "gene_symbol": "PUF60",
  "gene_name": "Poly(U)-binding-splicing factor PUF60"
}